positive regulation of non-motile cilium assembly [GO:1902857] (biological process) Relationships: is a type of positive regulation of cilium assembly [GO:0045724]; is a type of regulation of non-motile cilium assembly [GO:1902855]; positively regulates non-motile cilium assembly [GO:1905515] Also known as: activation of immotile primary cilium assembly, activation of nonmotile primary cilium assembly, activation of sensory cilium assembly, activation of nonmotile primary cilia assembly, activation of sensory cilium biogenesis, positive regulation of immotile primary cilium assembly, positive regulation of nonmotile primary cilia assembly, positive regulation of nonmotile primary cilium assembly, positive regulation of sensory cilium assembly, positive regulation of sensory cilium biogenesis, up regulation of immotile primary cilium assembly, up regulation of nonmotile primary cilia assembly, up regulation of nonmotile primary cilium assembly, up regulation of sensory cilium assembly, up regulation of sensory cilium biogenesis, up-regulation of immotile primary cilium assembly, up-regulation of nonmotile primary cilia assembly, up-regulation of nonmotile primary cilium assembly, up-regulation of sensory cilium assembly, up-regulation of sensory cilium biogenesis, upregulation of immotile primary cilium assembly, upregulation of nonmotile primary cilia assembly, upregulation of nonmotile primary cilium assembly, upregulation of sensory cilium assembly, upregulation of sensory cilium biogenesis Definition: Any process that activates or increases the frequency, rate or extent of non-motile cilium assembly. References: PMID:23807208 Sources: GOC:TermGenie, GOC:cilia, GOC:kmv, GO_REF:0000058